{
  "gene": "UniProtKB:Q9P0R6",
  "term_id": "GO:0019207",
  "gene_symbol": "GSKIP",
  "term_label": "kinase regulator activity",
  "gene_name": "GSK3B-interacting protein"
}